{
  "gene_symbol": "NEDD4",
  "gene_name": "E3 ubiquitin-protein ligase NEDD4",
  "term_label": "ubiquitin-dependent protein catabolic process",
  "term_id": "GO:0006511",
  "gene": "UniProtKB:P46934"
}